S-(hydroxymethyl)glutathione synthase activity [GO:0051907] (molecular function) Definition: Catalysis of the reaction: S-(hydroxymethyl)glutathione = formaldehyde + glutathione. Also known as: glutathione-dependent formaldehyde-activating enzyme activity, Gfa, S-(hydroxymethyl)glutathione formaldehyde-lyase (glutathione-forming), S-(hydroxymethyl)glutathione formaldehyde-lyase activity Relationships: is a type of GO:0016846 Sources: EC:4.4.1.22, RHEA:22488